regulation of dopamine metabolic process [GO:0042053] (biological process) Definition: Any process that modulates the frequency, rate or extent of the chemical reactions and pathways involving dopamine. Subtypes: negative regulation of dopamine metabolic process [GO:0045963], GO:0045964, regulation of dopamine biosynthetic process [GO:1903179] Relationships: is a type of regulation of catecholamine metabolic process [GO:0042069]; regulates dopamine metabolic process [GO:0042417] Also known as: regulation of dopamine metabolism Sources: GOC:go_curators